{
  "term_label": "immune response",
  "gene_name": "Immunoglobulin kappa variable 1D-39",
  "gene": "UniProtKB:P04432",
  "term_id": "GO:0006955",
  "gene_symbol": "IGKV1D-39"
}